{
  "gene_name": "2'-5'-oligoadenylate synthase-like protein",
  "gene_symbol": "OASL",
  "term_label": "double-stranded RNA binding",
  "term_id": "GO:0003725",
  "gene": "UniProtKB:Q15646"
}